melibiose catabolic process [GO:0005995] (BP) Definition: The chemical reactions and pathways resulting in the breakdown of melibiose, the disaccharide 6-O-alpha-D-galactopyranosyl-D-glucose. Sources: ISBN:0198547684 Relationships: is a type of disaccharide catabolic process [GO:0046352] Also known as: melibiose breakdown, melibiose catabolism, melibiose degradation